{
  "gene": "UniProtKB:O43247",
  "term_id": "UNKNOWN:0002",
  "term_label": "Unknown biological process",
  "gene_symbol": "TEX33",
  "gene_name": "Testis-expressed protein 33"
}